{
  "gene_name": "Angiopoietin-related protein 4",
  "term_label": "enzyme inhibitor activity",
  "gene_symbol": "ANGPTL4",
  "term_id": "GO:0004857",
  "gene": "UniProtKB:Q9BY76"
}